antibacterial peptide secretion [GO:0002779] (biological process) Regulation: RO_0002211 by regulation of antibacterial peptide secretion [GO:0002797]; negatively regulated by negative regulation of antibacterial peptide secretion [GO:0002798]; RO_0002213 by positive regulation of antibacterial peptide secretion [GO:0002799] Relationships: is a type of antimicrobial peptide secretion [GO:0002776]; is part of GO:0002778 References: PMID:11807545, PMID:15638771 Sources: GOC:add, ISBN:0781735149 Definition: The regulated release of an antibacterial peptide from a cell or a tissue.